{
  "term_label": "positive regulation of cytokinesis",
  "gene_symbol": "CDC14A",
  "term_id": "GO:0032467",
  "gene_name": "Dual specificity protein phosphatase CDC14A",
  "gene": "UniProtKB:Q9UNH5"
}